{
  "term_label": "cell differentiation",
  "term_id": "GO:0030154",
  "gene_symbol": "SMAD4",
  "gene_name": "Mothers against decapentaplegic homolog 4",
  "gene": "UniProtKB:Q13485"
}